tryptophan 2'-dioxygenase activity [GO:0050360] (MF) Sources: EC:1.13.99.3, MetaCyc:TRYPTOPHAN-2-DIOXYGENASE-RXN Definition: Catalysis of the reaction: L-tryptophan + O2 = 3-indoleglycolaldehyde + CO2 + NH3. Relationships: is a type of oxidoreductase activity, acting on single donors with incorporation of molecular oxygen [GO:0016701] Also known as: L-tryptophan:oxygen 2'-oxidoreductase (side-chain-cleaving), TSO I, TSO II, TSO activity, indole-3-alkane alpha-hydroxylase activity, indolyl-3-alkan alpha-hydroxylase activity, tryptophan side chain oxidase II, tryptophan side chain oxidase activity, tryptophan side chain oxidase type I, tryptophan side-chain alpha,beta-oxidase activity, tryptophan side-chain oxidase activity